{
  "gene_symbol": "KRT7",
  "gene": "UniProtKB:P08729",
  "gene_name": "Keratin, type II cytoskeletal 7",
  "term_id": "GO:0031424",
  "term_label": "keratinization"
}